{
  "gene": "UniProtKB:Q9Y5X9",
  "term_label": "triglyceride catabolic process",
  "gene_symbol": "LIPG",
  "gene_name": "Endothelial lipase",
  "term_id": "GO:0019433"
}